{
  "term_id": "GO:0005634",
  "gene_symbol": "SALL3",
  "gene": "UniProtKB:Q9BXA9",
  "gene_name": "Sal-like protein 3",
  "term_label": "nucleus"
}